{
  "term_id": "UNKNOWN:0003",
  "gene_name": "Protein MEMO1",
  "gene_symbol": "MEMO1",
  "term_label": "Unknown cellular component",
  "gene": "UniProtKB:Q9Y316"
}